{
  "gene": "UniProtKB:Q99504",
  "gene_symbol": "EYA3",
  "term_label": "cell differentiation",
  "term_id": "GO:0030154",
  "gene_name": "Eyes absent homolog 3"
}